intronic box H/ACA snoRNA processing [GO:0034966] (biological process) Definition: Any process involved in the conversion of a primary box H/ACA type small nucleolar RNA (snoRNA) transcript that resides within, and is processed from, the intron of a pre-mRNA into a mature box H/ACA snoRNA. Sources: GOC:mah Relationships: is a type of intronic snoRNA processing [GO:0031070]; is a type of box H/ACA sno(s)RNA processing [GO:0034964]